{
  "gene_symbol": "MAP4K4",
  "term_label": "regulation of MAPK cascade",
  "gene": "UniProtKB:O95819",
  "gene_name": "Mitogen-activated protein kinase kinase kinase kinase 4",
  "term_id": "GO:0043408"
}